{
  "term_label": "Unknown biological process",
  "gene_symbol": "INO80D",
  "gene_name": "INO80 complex subunit D",
  "term_id": "UNKNOWN:0002",
  "gene": "UniProtKB:Q53TQ3"
}